{
  "gene_symbol": "KCNK3",
  "term_label": "potassium ion leak channel activity",
  "term_id": "GO:0022841",
  "gene": "UniProtKB:O14649",
  "gene_name": "Potassium channel subfamily K member 3"
}